regulation of sorocarp development [GO:0031156] (biological process) Subtypes: GO:1901261 Definition: Any process that modulates the frequency, rate or extent of sorocarp development. An example of this process is found in Dictyostelium discoideum. References: PMID:4332228 Sources: GOC:mah, GOC:mtg_sensu Also known as: regulation of fruiting body development, regulation of fruiting body formation Relationships: is a type of regulation of developmental process [GO:0050793]; RO_0002211 GO:0030587